{
  "gene_name": "Putative uncharacterized protein PRO0461",
  "term_label": "Unknown cellular component",
  "gene_symbol": "PRO0461",
  "gene": "UniProtKB:Q9UI25",
  "term_id": "UNKNOWN:0003"
}